{
  "term_id": "GO:0035023",
  "gene_symbol": "DOCK8",
  "gene": "UniProtKB:Q8NF50",
  "term_label": "regulation of Rho protein signal transduction",
  "gene_name": "Dedicator of cytokinesis protein 8"
}